{
  "gene": "UniProtKB:Q9BS31",
  "term_label": "DNA-binding transcription factor activity",
  "gene_name": "Zinc finger protein 649",
  "gene_symbol": "ZNF649",
  "term_id": "GO:0003700"
}